symbiont-mediated suppression of host type III interferon-mediated signaling pathway [GO:0140885] (biological process) Also known as: negative regulation by virus of host type III interferon-mediated signaling pathway, suppression by virus of host type III IFN-mediated signaling pathway, suppression by virus of host type III interferon-mediated signalling pathway, suppression by virus of host type III interferon-mediated signaling pathway Relationships: is a type of symbiont-mediated suppression of host interferon-mediated signaling pathway [GO:0140886] Definition: A process in which a symbiont interferes with, inhibits or disrupts a type III interferon-mediated signaling in the host organism. Type III interferon is also known as interferon-lambda. References: PMID:32464097